negative regulation of calcium ion transmembrane transport via high voltage-gated calcium channel [GO:1904878] (biological process) Relationships: is a type of GO:1902514; is a type of negative regulation of calcium ion transmembrane transport [GO:1903170]; negatively regulates calcium ion transmembrane transport via high voltage-gated calcium channel [GO:0061577] Also known as: down regulation of generation of L-type calcium current, down-regulation of generation of L-type calcium current, downregulation of generation of L-type calcium current, inhibition of generation of L-type calcium current, negative regulation of generation of L-type calcium current Definition: Any process that stops, prevents or reduces the frequency, rate or extent of calcium ion transmembrane transport via high voltage-gated calcium channel. References: PMID:23071515 Sources: GOC:TermGenie, GO_REF:0000058